{
  "term_label": "ubiquitin protein ligase activity",
  "gene": "UniProtKB:O60291",
  "gene_symbol": "MGRN1",
  "gene_name": "E3 ubiquitin-protein ligase MGRN1",
  "term_id": "GO:0061630"
}